{
  "term_id": "GO:0005739",
  "gene_name": "NADH dehydrogenase [ubiquinone] 1 alpha subcomplex assembly factor 4",
  "term_label": "mitochondrion",
  "gene_symbol": "NDUFAF4",
  "gene": "UniProtKB:Q9P032"
}